positive regulation of citrulline biosynthetic process [GO:1903250] (biological process) Also known as: positive regulation of citrulline anabolism, positive regulation of citrulline biosynthesis, positive regulation of citrulline formation, positive regulation of citrulline synthesis, up regulation of citrulline anabolism, up regulation of citrulline biosynthesis, up regulation of citrulline biosynthetic process, up regulation of citrulline formation, up regulation of citrulline synthesis, up-regulation of citrulline anabolism, up-regulation of citrulline biosynthesis, up-regulation of citrulline biosynthetic process, up-regulation of citrulline formation, up-regulation of citrulline synthesis, upregulation of citrulline anabolism, upregulation of citrulline biosynthesis, upregulation of citrulline biosynthetic process, upregulation of citrulline formation, upregulation of citrulline synthesis, activation of citrulline anabolism, activation of citrulline biosynthesis, activation of citrulline biosynthetic process, activation of citrulline formation, activation of citrulline synthesis Definition: Any process that activates or increases the frequency, rate or extent of citrulline biosynthetic process. References: PMID:19278978 Sources: GOC:BHF, GOC:TermGenie, GOC:rl, GO_REF:0000058 Relationships: is a type of GO:0062013; is a type of regulation of citrulline biosynthetic process [GO:1903248]; is a type of GO:2000284; positively regulates citrulline biosynthetic process [GO:0019240]